{
  "gene_symbol": "MUTYH",
  "term_id": "GO:0032357",
  "term_label": "oxidized purine DNA binding",
  "gene_name": "Adenine DNA glycosylase",
  "gene": "UniProtKB:Q9UIF7"
}